{
  "gene_symbol": "ZBTB45",
  "gene_name": "Zinc finger and BTB domain-containing protein 45",
  "gene": "UniProtKB:Q96K62",
  "term_label": "DNA-binding transcription repressor activity, RNA polymerase II-specific",
  "term_id": "GO:0001227"
}